{
  "term_label": "Unknown molecular function",
  "gene_symbol": "C8orf90",
  "gene_name": "Uncharacterized protein C8orf90",
  "gene": "UniProtKB:A0A2R8Y2Y2",
  "term_id": "UNKNOWN:0001"
}